{
  "term_id": "GO:0001618",
  "gene": "UniProtKB:Q96D42",
  "gene_name": "Hepatitis A virus cellular receptor 1",
  "term_label": "virus receptor activity",
  "gene_symbol": "HAVCR1"
}